{
  "term_label": "calcium-activated potassium channel activity",
  "term_id": "GO:0015269",
  "gene_symbol": "KCNMB2",
  "gene": "UniProtKB:Q9Y691",
  "gene_name": "Calcium-activated potassium channel subunit beta-2"
}